{
  "gene_symbol": "APOLD1",
  "term_id": "GO:0008289",
  "gene_name": "Apolipoprotein L domain-containing protein 1",
  "gene": "UniProtKB:Q96LR9",
  "term_label": "lipid binding"
}